{
  "gene": "UniProtKB:Q3SXY8",
  "gene_symbol": "ARL13B",
  "term_label": "non-motile cilium assembly",
  "term_id": "GO:1905515",
  "gene_name": "ADP-ribosylation factor-like protein 13B"
}